{
  "gene_symbol": "CD70",
  "gene_name": "CD70 antigen",
  "gene": "UniProtKB:P32970",
  "term_label": "plasma membrane",
  "term_id": "GO:0005886"
}